myocardial epithelial involution involved in heart jogging [GO:0003304] (biological process) Definition: The morphogenetic process in which the myocardium bends along a linear axis and contributes to the process of heart jogging. Relationships: is a type of morphogenesis of an epithelial fold [GO:0060571]; is part of heart jogging [GO:0003146] Sources: GOC:mtg_heart